plastoquinone biosynthetic process [GO:0010236] (biological process) Definition: The chemical reactions and pathways resulting in the formation of plastoquinone, a lipid-soluble electron-transporting coenzyme present in the chloroplast. Sources: GOC:sm Also known as: plastoquinone anabolism, plastoquinone biosynthesis, plastoquinone formation, plastoquinone synthesis Relationships: is a type of quinone biosynthetic process [GO:1901663]